negative regulation of synaptic transmission, glutamatergic [GO:0051967] (biological process) Sources: GOC:ai Relationships: is_a negative regulation of synaptic transmission [GO:0050805]; is_a regulation of synaptic transmission, glutamatergic [GO:0051966]; negatively regulates GO:0035249 Subtypes: negative regulation of glutamate secretion, neurotransmission [GO:1903295] Also known as: down regulation of synaptic transmission, glutamatergic, down-regulation of synaptic transmission, glutamatergic, downregulation of synaptic transmission, glutamatergic, inhibition of synaptic transmission, glutamatergic Definition: Any process that stops, prevents, or reduces the frequency, rate or extent of glutamatergic synaptic transmission, the process of communication from a neuron to another neuron across a synapse using the neurotransmitter glutamate.